thymic T cell selection [GO:0045061] (biological process) Definition: The process of T cell selection that occurs in the thymus. References: PMID:12414722 Sources: ISBN:0781735149 Also known as: thymic T lymphocyte selection, thymic T-cell selection, thymic T-lymphocyte selection Relationships: is a type of T cell selection [GO:0045058]; is part of T cell differentiation in thymus [GO:0033077] Subtypes: positive thymic T cell selection [GO:0045059], negative thymic T cell selection [GO:0045060]